{
  "gene_name": "Gap junction alpha-1 protein",
  "term_label": "connexin complex",
  "term_id": "GO:0005922",
  "gene": "UniProtKB:P17302",
  "gene_symbol": "GJA1"
}